{
  "term_label": "Unknown biological process",
  "gene_name": "Deoxyguanosine kinase, mitochondrial",
  "gene_symbol": "DGUOK",
  "gene": "UniProtKB:Q16854",
  "term_id": "UNKNOWN:0002"
}